{
  "gene_symbol": "GNAT2",
  "gene": "UniProtKB:P19087",
  "gene_name": "Guanine nucleotide-binding protein G(t) subunit alpha-2",
  "term_label": "heterotrimeric G-protein complex",
  "term_id": "GO:0005834"
}